replication fork protection complex [GO:0031298] (cellular component) References: PMID:12944972, PMID:15367656, PMID:19819872 Also known as: FPC, fork pausing complex, Swi1-Swi3 complex, TIMELESS-TIPIN complex Definition: A heterotrimeric replication-pausing complex conserved in eukaryotes and associated with the replication fork; the complex stabilizes stalled replication forks and is thought to be involved in coordinating leading- and lagging-strand synthesis and in replication checkpoint signaling. Required for maximal fork speed both in vivo and in vitro. Relationships: is a type of nuclear protein-containing complex [GO:0140513]; is part of nuclear replication fork [GO:0043596]